poly(hydroxyalkanoate) biosynthetic process from fatty acid [GO:1902925] (biological process) Relationships: is a type of fatty acid metabolic process [GO:0006631]; is a type of GO:1901441 Also known as: poly(hydroxyalkanoate) anabolism from fatty acid, poly(hydroxyalkanoate) biosynthesis from fatty acid, poly(hydroxyalkanoate) formation from fatty acid, poly(hydroxyalkanoate) synthesis from fatty acid Definition: The chemical reactions and pathways resulting in the formation of poly(hydroxyalkanoate) from fatty acid. References: PMID:21129764 Sources: GOC:TermGenie, GOC:mengo_curators, GO_REF:0000092